{
  "term_id": "UNKNOWN:0001",
  "gene_symbol": "IRX2-DT",
  "gene": "UniProtKB:Q86SI9",
  "term_label": "Unknown molecular function",
  "gene_name": "Putative uncharacterized protein IRX2-DT"
}